interleukin-35 complex [GO:0070745] (cellular component) Also known as: IL-35 complex, EBI3, IL12A, p35 References: PMID:19161428, PMID:19161429 Sources: GOC:add Relationships: is a type of protein-containing complex [GO:0032991]; is part of extracellular space [GO:0005615] Note: Note that this heterodimeric cytokine utilizes the same IL-12p35 subunit as its alpha chain as IL-12 uses and the same EBI3 subunit (product of EBI3, Epstein-Barr virus induced gene 3) as its beta chain as IL-27 uses. IL-35 requires both subunits -- there is no separate IL35 gene. Definition: A protein complex that is composed of an interleukin-12 alpha subunit (p35, product of the IL12A gene) and an EBI3 subunit and is secreted into the extracellular space.